{
  "gene": "UniProtKB:Q92922",
  "gene_symbol": "SMARCC1",
  "term_label": "histone binding",
  "term_id": "GO:0042393",
  "gene_name": "SWI_SNF complex subunit SMARCC1"
}